{
  "gene_name": "Sperm-associated antigen 17",
  "term_label": "Unknown molecular function",
  "gene_symbol": "SPAG17",
  "gene": "UniProtKB:Q6Q759",
  "term_id": "UNKNOWN:0001"
}